{
  "gene_symbol": "LONRF2",
  "term_label": "Unknown cellular component",
  "gene_name": "LON peptidase N-terminal domain and RING finger protein 2",
  "gene": "UniProtKB:Q1L5Z9",
  "term_id": "UNKNOWN:0003"
}